{
  "term_label": "Unknown biological process",
  "gene_symbol": "NUP37",
  "gene": "UniProtKB:Q8NFH4",
  "term_id": "UNKNOWN:0002",
  "gene_name": "Nucleoporin Nup37"
}